syntaxin-1 binding [GO:0017075] (molecular function) Definition: Binding to a syntaxin-1 SNAP receptor. Relationships: is a type of GO:0019905 Sources: GOC:ai